{
  "gene_name": "E3 ubiquitin-protein ligase MARCHF6",
  "term_id": "GO:0043161",
  "gene_symbol": "MARCHF6",
  "gene": "UniProtKB:O60337",
  "term_label": "proteasome-mediated ubiquitin-dependent protein catabolic process"
}